{
  "gene_name": "BRCA1-A complex subunit RAP80",
  "gene_symbol": "UIMC1",
  "term_label": "histone binding",
  "gene": "UniProtKB:Q96RL1",
  "term_id": "GO:0042393"
}